{
  "term_label": "intrinsic apoptotic signaling pathway in response to DNA damage by p53 class mediator",
  "term_id": "GO:0042771",
  "gene": "UniProtKB:Q86Z02",
  "gene_symbol": "HIPK1",
  "gene_name": "Homeodomain-interacting protein kinase 1"
}